{
  "gene_symbol": "PIGV",
  "term_id": "GO:0031501",
  "term_label": "mannosyltransferase complex",
  "gene_name": "GPI mannosyltransferase 2",
  "gene": "UniProtKB:Q9NUD9"
}